{
  "term_id": "GO:0002221",
  "gene_name": "Nucleotide-binding oligomerization domain-containing protein 2",
  "gene": "UniProtKB:Q9HC29",
  "gene_symbol": "NOD2",
  "term_label": "pattern recognition receptor signaling pathway"
}